{
  "term_label": "cytoplasm",
  "gene_symbol": "WWP1",
  "gene_name": "NEDD4-like E3 ubiquitin-protein ligase WWP1",
  "gene": "UniProtKB:Q9H0M0",
  "term_id": "GO:0005737"
}